{
  "gene_name": "Male-specific lethal 1 homolog",
  "term_id": "GO:0006338",
  "term_label": "chromatin remodeling",
  "gene_symbol": "MSL1",
  "gene": "UniProtKB:Q68DK7"
}